{
  "gene_symbol": "KLHL13",
  "term_id": "GO:0032465",
  "gene_name": "Kelch-like protein 13",
  "term_label": "regulation of cytokinesis",
  "gene": "UniProtKB:Q9P2N7"
}